{
  "term_label": "gamma-aminobutyric acid catabolic process",
  "gene_name": "4-aminobutyrate aminotransferase, mitochondrial",
  "gene": "UniProtKB:P80404",
  "term_id": "GO:0009450",
  "gene_symbol": "ABAT"
}